myelination in peripheral nervous system [GO:0022011] (biological process) Relationships: is a type of GO:0032292; is a type of myelination [GO:0042552]; is part of GO:0014044 Sources: GOC:cls, GOC:dgh, GOC:dph, GOC:jid, GO_REF:0000021 Definition: The process in which neuronal axons and dendrites become coated with a segmented lipid-rich sheath (myelin) to enable faster and more energetically efficient conduction of electrical impulses. The sheath is formed by the cell membranes of Schwann cells in the peripheral nervous system. Adjacent myelin segments are separated by a non-myelinated stretch of axon called a node of Ranvier. Also known as: peripheral nervous system myelination